{
  "term_id": "GO:0022841",
  "gene_name": "Endosomal_lysosomal proton channel TMEM175",
  "gene": "UniProtKB:Q9BSA9",
  "gene_symbol": "TMEM175",
  "term_label": "potassium ion leak channel activity"
}